{
  "term_label": "kinase activity",
  "gene_symbol": "FN3K",
  "gene_name": "Fructosamine-3-kinase",
  "gene": "UniProtKB:Q9H479",
  "term_id": "GO:0016301"
}